{
  "gene_symbol": "KCNA4",
  "gene_name": "Potassium voltage-gated channel subfamily A member 4",
  "term_id": "GO:0001508",
  "term_label": "action potential",
  "gene": "UniProtKB:P22459"
}